{
  "term_id": "GO:0006465",
  "gene_name": "Signal peptidase complex catalytic subunit SEC11C",
  "gene": "UniProtKB:Q9BY50",
  "gene_symbol": "SEC11C",
  "term_label": "signal peptide processing"
}